{
  "gene_name": "Bone morphogenetic protein 8B",
  "term_label": "extracellular space",
  "term_id": "GO:0005615",
  "gene": "UniProtKB:P34820",
  "gene_symbol": "BMP8B"
}